{
  "term_label": "presynaptic active zone",
  "term_id": "GO:0048786",
  "gene_symbol": "PNISR",
  "gene": "UniProtKB:Q8TF01",
  "gene_name": "Arginine_serine-rich protein PNISR"
}